{
  "gene_symbol": "ZNF34",
  "gene": "UniProtKB:Q8IZ26",
  "term_id": "GO:0006357",
  "term_label": "regulation of transcription by RNA polymerase II",
  "gene_name": "Zinc finger protein 34"
}